adenosine biosynthetic process [GO:0046086] (biological process) Also known as: adenosine anabolism, adenosine biosynthesis, adenosine formation, adenosine synthesis Subtypes: adenosine salvage [GO:0006169] Definition: The chemical reactions and pathways resulting in the formation of adenosine, adenine riboside, a ribonucleoside found widely distributed in cells of every type as the free nucleoside and in combination in nucleic acids and various nucleoside coenzymes. Sources: GOC:go_curators Relationships: is_a adenosine metabolic process [GO:0046085]; is a type of purine ribonucleoside biosynthetic process [GO:0046129]